{
  "gene_symbol": "CSNKA2IP",
  "term_id": "UNKNOWN:0001",
  "gene_name": "Casein kinase II subunit alpha'-interacting protein",
  "term_label": "Unknown molecular function",
  "gene": "UniProtKB:A0A1B0GTH6"
}